{
  "gene_symbol": "SIKE1",
  "gene": "UniProtKB:Q9BRV8",
  "term_id": "UNKNOWN:0001",
  "gene_name": "Suppressor of IKBKE 1",
  "term_label": "Unknown molecular function"
}